cellular response to isooctane [GO:1902789] (biological process) Relationships: is a type of cellular response to alkane [GO:1902779]; is a type of response to isooctane [GO:1902788] Definition: Any process that results in a change in state or activity of a cell (in terms of movement, secretion, enzyme production, gene expression, etc.) as a result of an isooctane stimulus. References: PMID:22328008 Sources: GOC:TermGenie, GOC:mengo_curators, GO_REF:0000071